{
  "gene_name": "PiggyBac transposable element-derived protein 5",
  "term_id": "GO:0004803",
  "gene": "UniProtKB:Q8N414",
  "gene_symbol": "PGBD5",
  "term_label": "transposase activity"
}